deoxycytidine salvage [GO:0006237] (biological process) Definition: Any process that generates deoxycytidine, 2-deoxyribosylcytosine, from derivatives of it, without de novo synthesis. Relationships: is a type of pyrimidine deoxyribonucleoside salvage [GO:0043099]; is a type of GO:0046093 Sources: GOC:jl